ajmaline biosynthetic process [GO:1900988] (biological process) Definition: The chemical reactions and pathways resulting in the formation of ajmaline. Sources: GOC:TermGenie, GOC:yaf Also known as: ajmaline metabolic process, ajmaline metabolism, ajmaline anabolism, ajmaline biosynthesis, ajmaline formation, ajmaline synthesis Relationships: is a type of GO:0009709